{
  "term_id": "GO:0005886",
  "gene": "UniProtKB:P48146",
  "term_label": "plasma membrane",
  "gene_symbol": "NPBWR2",
  "gene_name": "Neuropeptides B_W receptor type 2"
}